adenylate cyclase-inhibiting G protein-coupled glutamate receptor signaling pathway [GO:0007196] (biological process) Relationships: is a type of adenylate cyclase-inhibiting G protein-coupled receptor signaling pathway [GO:0007193]; is a type of G protein-coupled glutamate receptor signaling pathway [GO:0007216]; has part adenylate cyclase inhibiting G protein-coupled glutamate receptor activity [GO:0001640] Definition: An adenylate cyclase-inhibiting G protein-coupled receptor signaling pathway initiated by glutamate binding to its receptor, and ending with the regulation of a downstream cellular process. Sources: GOC:dph, GOC:mah, GOC:signaling, GOC:tb Also known as: adenylate cyclase-inhibiting G-protein coupled glutamate receptor signaling pathway, inhibition of adenylate cyclase activity by metabotropic glutamate receptor signaling pathway, inhibition of adenylate cyclase activity by metabotropic glutamate receptor signalling pathway, metabotropic glutamate receptor, adenylate cyclase inhibiting pathway, metabotropic glutamate receptor, adenylyl cyclase inhibiting pathway, inhibition of adenylate cyclase activity by G-protein-coupled glutamate receptor signaling pathway